{
  "gene": "UniProtKB:Q5XKR9",
  "term_label": "Unknown molecular function",
  "gene_symbol": "FAM104B",
  "gene_name": "Protein FAM104B",
  "term_id": "UNKNOWN:0001"
}